{
  "term_id": "GO:0008157",
  "gene_name": "Protein phosphatase 1 regulatory subunit 3A",
  "term_label": "protein phosphatase 1 binding",
  "gene_symbol": "PPP1R3A",
  "gene": "UniProtKB:Q16821"
}